{
  "gene_symbol": "CLCN4",
  "gene_name": "H(+)_Cl(-) exchange transporter 4",
  "gene": "UniProtKB:P51793",
  "term_id": "GO:0005769",
  "term_label": "early endosome"
}